{
  "term_id": "GO:0000978",
  "term_label": "RNA polymerase II cis-regulatory region sequence-specific DNA binding",
  "gene_symbol": "SNAI2",
  "gene": "UniProtKB:O43623",
  "gene_name": "Zinc finger protein SNAI2"
}